{
  "gene_symbol": "LMNB2",
  "gene": "UniProtKB:Q03252",
  "term_label": "structural constituent of cytoskeleton",
  "term_id": "GO:0005200",
  "gene_name": "Lamin-B2"
}